{
  "gene_symbol": "CYB561A3",
  "gene_name": "Lysosomal membrane ascorbate-dependent ferrireductase CYB561A3",
  "gene": "UniProtKB:Q8NBI2",
  "term_id": "GO:0016491",
  "term_label": "oxidoreductase activity"
}